{
  "gene_symbol": "UNQ6126_PRO20091",
  "gene": "UniProtKB:Q6UXV3",
  "term_label": "Unknown cellular component",
  "gene_name": "Uncharacterized protein UNQ6126_PRO20091",
  "term_id": "UNKNOWN:0003"
}